{
  "gene": "UniProtKB:Q9Y6V0",
  "gene_symbol": "PCLO",
  "term_id": "GO:0030424",
  "gene_name": "Protein piccolo",
  "term_label": "axon"
}